{
  "gene": "UniProtKB:Q01415",
  "term_label": "galactose metabolic process",
  "term_id": "GO:0006012",
  "gene_symbol": "GALK2",
  "gene_name": "N-acetylgalactosamine kinase"
}